{
  "term_label": "sarcolemma",
  "gene_symbol": "ALOX12",
  "gene_name": "Polyunsaturated fatty acid lipoxygenase ALOX12",
  "term_id": "GO:0042383",
  "gene": "UniProtKB:P18054"
}